{
  "term_id": "GO:0030527",
  "gene_name": "Histone H2B type 1-L",
  "term_label": "structural constituent of chromatin",
  "gene": "UniProtKB:Q99880",
  "gene_symbol": "H2BC13"
}